metanephric short nephron development [GO:0072270] (biological process) Definition: The process whose specific outcome is the progression of a short nephron in the metanephros over time, from its formation to the mature structure. Short nephrons are associated with mid-cortical and superficial glomeruli, are situated entirely in the outer medulla, and have no thin ascending limb. Relationships: is a type of short nephron development [GO:0072030]; is a type of metanephric nephron development [GO:0072210] Sources: GOC:mtg_kidney_jan10